{
  "gene_symbol": "PRR25",
  "gene": "UniProtKB:Q96S07",
  "term_id": "UNKNOWN:0001",
  "gene_name": "Proline-rich protein 25",
  "term_label": "Unknown molecular function"
}